{
  "term_label": "endoplasmic reticulum membrane",
  "gene": "UniProtKB:Q96Q80",
  "gene_symbol": "DERL3",
  "term_id": "GO:0005789",
  "gene_name": "Derlin-3"
}